{
  "gene_name": "Interferon alpha-5",
  "gene": "UniProtKB:P01569",
  "gene_symbol": "IFNA5",
  "term_label": "type I interferon-mediated signaling pathway",
  "term_id": "GO:0060337"
}